{
  "gene": "UniProtKB:P35408",
  "gene_symbol": "PTGER4",
  "term_id": "GO:0006954",
  "gene_name": "Prostaglandin E2 receptor EP4 subtype",
  "term_label": "inflammatory response"
}